{
  "term_id": "GO:0005737",
  "gene": "UniProtKB:P56524",
  "gene_name": "Histone deacetylase 4",
  "gene_symbol": "HDAC4",
  "term_label": "cytoplasm"
}